{
  "gene": "UniProtKB:Q9H426",
  "term_id": "UNKNOWN:0001",
  "gene_symbol": "RIMS4",
  "term_label": "Unknown molecular function",
  "gene_name": "Regulating synaptic membrane exocytosis protein 4"
}